{
  "term_label": "structural constituent of ribosome",
  "gene_symbol": "RPS24",
  "gene": "UniProtKB:P62847",
  "gene_name": "Small ribosomal subunit protein eS24",
  "term_id": "GO:0003735"
}